{
  "gene_symbol": "CSAD",
  "term_label": "taurine biosynthetic process",
  "term_id": "GO:0042412",
  "gene": "UniProtKB:Q9Y600",
  "gene_name": "Cysteine sulfinic acid decarboxylase"
}